chemokine (C-C motif) ligand 11 production [GO:0071954] (biological process) References: PMID:9600955 Sources: GOC:mah Relationships: is a type of chemokine production [GO:0032602] Definition: The appearance of chemokine (C-C motif) ligand 11 (CCL11, also known as eotaxin-1) due to biosynthesis or secretion following a cellular stimulus, resulting in an increase in its intracellular or extracellular levels. Also known as: eotaxin production, C-C motif chemokine 11 production, CCL-11 production, CCL11 production, eotaxin-1 production